P-type ion transporter activity [GO:0015662] (molecular function) References: PMID:10322420, PMID:10600683 Relationships: is a type of P-type transmembrane transporter activity [GO:0140358] Definition: Enables the transfer of a solute or solutes from one side of a membrane to the other according to the reaction: ATP + H2O = ADP + phosphate, to directly drive the transport of ions across a membrane. The reaction is characterized by the transient formation of a high-energy aspartyl-phosphoryl-enzyme intermediate. Subtypes: GO:0005388, P-type cadmium transporter activity [GO:0008551], P-type proton-exporting transporter activity [GO:0008553], P-type sodium transporter activity [GO:0008554], P-type potassium transmembrane transporter activity [GO:0008556], GO:0015444, P-type silver transporter activity [GO:0015445], P-type zinc transporter activity [GO:0016463], P-type cobalt transporter activity [GO:0032778], GO:0043682, GO:0140581, GO:0140613 Also known as: ATPase activity, coupled to transmembrane movement of ions, phosphorylative mechanism, P-type ATPase activity, zinc, cadmium, cobalt, nickel, lead-efflux ATPase activity, ion transmembrane transporter activity, phosphorylative mechanism